flavin-containing compound biosynthetic process [GO:0042727] (biological process) Relationships: is a type of biosynthetic process [GO:0009058]; is a type of GO:0042726 Also known as: flavin-containing compound anabolism, flavin-containing compound biosynthesis, flavin-containing compound formation, flavin-containing compound synthesis, riboflavin and derivative biosynthesis, riboflavin and derivative biosynthetic process, vitamin B2 and derivative biosynthesis, vitamin B2 and derivative biosynthetic process Subtypes: riboflavin biosynthetic process [GO:0009231], FMN biosynthetic process [GO:0009398], flavin adenine dinucleotide biosynthetic process [GO:0072388], prenyl-FMNH2 biosynthetic process [GO:0120232] Definition: The chemical reactions and pathways resulting in the formation of a flavin, any derivative of the dimethylisoalloxazine (7,8-dimethylbenzo[g]pteridine-2,4(3H,10H)-dione) skeleton, with a substituent on the 10 position. Sources: GOC:jl, GOC:mah